{
  "term_label": "D1 dopamine receptor binding",
  "gene": "UniProtKB:Q5JWF2",
  "gene_name": "Guanine nucleotide-binding protein G(s) subunit alpha isoforms XLas",
  "term_id": "GO:0031748",
  "gene_symbol": "GNAS"
}